{
  "term_label": "keratin filament",
  "gene_name": "Keratin, type II cytoskeletal 4",
  "gene_symbol": "KRT4",
  "term_id": "GO:0045095",
  "gene": "UniProtKB:P19013"
}